glycine catabolic process [GO:0006546] (biological process) Sources: GOC:go_curators Subtypes: GO:0019464, anaerobic glycine catabolic process [GO:0019669], glycine catabolic process to isobutanol [GO:1902696] Definition: The chemical reactions and pathways resulting in the breakdown of glycine, aminoethanoic acid. Relationships: is a type of glycine metabolic process [GO:0006544]; is a type of proteinogenic amino acid catabolic process [GO:0170040]; is a type of alpha-amino acid catabolic process [GO:1901606] Also known as: glycine breakdown, glycine catabolism, glycine degradation